{
  "gene_symbol": "NUDT5",
  "term_id": "GO:0019693",
  "gene": "UniProtKB:Q9UKK9",
  "gene_name": "ADP-sugar pyrophosphatase",
  "term_label": "ribose phosphate metabolic process"
}